(R)-6-hydroxynicotine oxidase activity [GO:0018530] (molecular function) Sources: EC:1.5.3.6, RHEA:10012 Relationships: is a type of hydroxy-nicotine oxidase activity [GO:0019116] Definition: Catalysis of the reaction: (R)-6-hydroxynicotine + H2O + O2 = 6-hydroxypseudooxynicotine + H2O2. Also known as: 6-hydroxy-D-nicotine oxidase activity, (R)-6-hydroxynicotine:oxygen oxidoreductase activity, D-6-hydroxynicotine oxidase activity